{
  "gene_symbol": "STARD8",
  "gene": "UniProtKB:Q92502",
  "term_id": "GO:0035023",
  "term_label": "regulation of Rho protein signal transduction",
  "gene_name": "StAR-related lipid transfer protein 8"
}